{
  "term_label": "Unknown cellular component",
  "gene_name": "BTB_POZ domain-containing protein KCTD18",
  "term_id": "UNKNOWN:0003",
  "gene_symbol": "KCTD18",
  "gene": "UniProtKB:Q6PI47"
}